{
  "term_label": "intracellular signal transduction",
  "gene": "UniProtKB:O96013",
  "gene_name": "Serine_threonine-protein kinase PAK 4",
  "gene_symbol": "PAK4",
  "term_id": "GO:0035556"
}